{
  "term_label": "glyoxylate metabolic process",
  "gene": "UniProtKB:Q5T013",
  "term_id": "GO:0046487",
  "gene_symbol": "HYI",
  "gene_name": "Putative hydroxypyruvate isomerase"
}